{
  "gene_name": "Zinc finger protein 333",
  "gene": "UniProtKB:Q96JL9",
  "term_label": "nucleus",
  "gene_symbol": "ZNF333",
  "term_id": "GO:0005634"
}